{
  "term_label": "transcription coactivator activity",
  "gene_name": "Steroid receptor RNA activator 1",
  "term_id": "GO:0003713",
  "gene_symbol": "SRA1",
  "gene": "UniProtKB:Q9HD15"
}